{
  "gene_symbol": "JAGN1",
  "term_id": "GO:0016192",
  "term_label": "vesicle-mediated transport",
  "gene_name": "Protein jagunal homolog 1",
  "gene": "UniProtKB:Q8N5M9"
}